{
  "gene": "UniProtKB:P14209",
  "gene_symbol": "CD99",
  "gene_name": "CD99 antigen",
  "term_id": "UNKNOWN:0001",
  "term_label": "Unknown molecular function"
}